{
  "gene_symbol": "COMMD3",
  "gene_name": "COMM domain-containing protein 3",
  "term_id": "UNKNOWN:0002",
  "term_label": "Unknown biological process",
  "gene": "UniProtKB:Q9UBI1"
}